T-helper cell differentiation [GO:0042093] (biological process) Definition: The process in which a relatively unspecialized thymocyte acquires specialized features of a T-helper cell. Sources: GOC:ebc Also known as: helper T cell differentiation, T-helper cell development Relationships: is a type of CD4-positive, alpha-beta T cell differentiation involved in immune response [GO:0002294] Subtypes: GO:0045063, T-helper 2 cell differentiation [GO:0045064], T follicular helper cell differentiation [GO:0061470], GO:0072539 Regulation: regulated by regulation of T-helper cell differentiation [GO:0045622]; negatively regulated by negative regulation of T-helper cell differentiation [GO:0045623]; positively regulated by GO:0045624